{
  "term_label": "signal transduction",
  "term_id": "GO:0007165",
  "gene": "UniProtKB:Q96GM1",
  "gene_name": "Phospholipid phosphatase-related protein type 2",
  "gene_symbol": "PLPPR2"
}